Ctf18 RFC-like complex [GO:0031390] (cellular component) Also known as: Ctf18-RFC, Ctf18-RLC, RFC (Ctf18) Relationships: is a type of GO:0140513; is part of GO:0005694 Definition: A heptameric complex related to replication factor C, which loads the DNA polymerase processivity factor proliferating cell nuclear antigen (PCNA) onto DNA and plays a vital role in chromosome cohesion. In Saccharomyces the subunits are known as Ctf18p, Rfc2p, Rfc3p, Rfc4p, Rfc5p, Dcc1p, and Ctf8p. References: PMID:14614842